{
  "term_id": "GO:1990573",
  "gene_name": "G protein-activated inward rectifier potassium channel 3",
  "gene": "UniProtKB:Q92806",
  "gene_symbol": "KCNJ9",
  "term_label": "potassium ion import across plasma membrane"
}